galactan 1,3-beta-galactosidase activity [GO:0033943] (molecular function) Definition: Catalysis of the hydrolysis of terminal, non-reducing beta-D-galactose residues in (1->3)-beta-D-galactopyranans. Sources: EC:3.2.1.145 Relationships: is a type of beta-galactosidase activity [GO:0004565] Also known as: galactan (1,3)-beta-D-galactosidase activity, galactan (1->3)-beta-D-galactosidase activity